{
  "gene_symbol": "ACOX1",
  "gene_name": "Peroxisomal acyl-coenzyme A oxidase 1",
  "term_label": "long-chain fatty acyl-CoA oxidase activity",
  "term_id": "GO:0120524",
  "gene": "UniProtKB:Q15067"
}